{
  "term_label": "cilium assembly",
  "gene": "UniProtKB:Q2TAC2",
  "term_id": "GO:0060271",
  "gene_symbol": "CCDC57",
  "gene_name": "Coiled-coil domain-containing protein 57"
}